(+)-neomenthol dehydrogenase activity [GO:0047501] (molecular function) Definition: Catalysis of the reaction: (+)-neomenthol + NADP+ = (2S,5R)-menthone + H+ + NADPH. Relationships: is a type of oxidoreductase activity, acting on the CH-OH group of donors, NAD or NADP as acceptor [GO:0016616] Sources: EC:1.1.1.208, RHEA:23812 Also known as: monoterpenoid dehydrogenase activity, (+)-neomenthol:NADP+ oxidoreductase activity